{
  "term_id": "GO:0060271",
  "gene": "UniProtKB:Q9NVD7",
  "gene_symbol": "PARVA",
  "term_label": "cilium assembly",
  "gene_name": "Alpha-parvin"
}